{
  "term_id": "GO:0045944",
  "gene": "UniProtKB:Q8NDY6",
  "gene_symbol": "BHLHE23",
  "gene_name": "Class E basic helix-loop-helix protein 23",
  "term_label": "positive regulation of transcription by RNA polymerase II"
}